phytochelatin transmembrane transport [GO:0071994] (BP) Note: Note that this term is not intended for use in annotating lateral movement within membranes. Subtypes: GO:0071995 Sources: GOC:mah, ISBN:0198506732 Also known as: phytochelatin membrane transport, cadystin transmembrane transport Definition: The process in which a phytochelatin is transported across a membrane. Phytochelatins are a group of peptides that bind metals (Cd, Zn, Cu, Pb, Hg) in thiolate coordination complexes. Relationships: is a type of transmembrane transport [GO:0055085]; is a type of phytochelatin transport [GO:0071993]